{
  "gene_name": "Urocortin",
  "term_id": "UNKNOWN:0001",
  "term_label": "Unknown molecular function",
  "gene": "UniProtKB:P55089",
  "gene_symbol": "UCN"
}